{
  "gene_name": "Acetylcholine receptor subunit beta",
  "term_label": "monoatomic ion transmembrane transport",
  "gene_symbol": "CHRNB1",
  "gene": "UniProtKB:P11230",
  "term_id": "GO:0034220"
}